{
  "term_id": "GO:0002250",
  "gene_name": "Interferon alpha-4",
  "gene_symbol": "IFNA4",
  "gene": "UniProtKB:P05014",
  "term_label": "adaptive immune response"
}